chondroitin sulfate proteoglycan binding [GO:0035373] (molecular function) Relationships: is a type of proteoglycan binding [GO:0043394] Sources: GOC:kmv, ISBN:0198506732 Definition: Binding to a chondroitin sulfate proteoglycan, any proteoglycan containing chondroitin sulfate as the glycosaminoglycan carbohydrate unit.